{
  "term_id": "GO:0031902",
  "term_label": "late endosome membrane",
  "gene_symbol": "GOSR2",
  "gene": "UniProtKB:O14653",
  "gene_name": "Golgi SNAP receptor complex member 2"
}